myosin VII complex [GO:0031477] (CC) References: PMID:28660889 Relationships: is a type of unconventional myosin complex [GO:0016461] Definition: A myosin complex containing a dimer of class VII myosin heavy chains and associated light chains. Myosin VII (240 kDa) is predicted to be a dimeric molecule with 5 IQ motifs and a tail region with a short stretch of coiled coil followed by two myosin-tail homology (MyTH4) domains, two talin-binding (FERM) domains and an SH3-domain.